lipid antigen assembly with MHC class Ib protein complex [GO:0002493] (biological process) Definition: The binding of a lipid antigen to the antigen binding groove of an MHC class Ib protein complex. Class Ib here refers to non-classical class I molecules, such as those of the CD1 gene family. References: PMID:15928678, PMID:15928680 Sources: GOC:add Relationships: is a type of protein-lipid complex assembly [GO:0065005]; is part of MHC class Ib protein complex assembly [GO:0002398]; is part of antigen processing and presentation of lipid antigen via MHC class Ib [GO:0048003]